{
  "gene": "UniProtKB:Q0D2H9",
  "gene_symbol": "GOLGA8DP",
  "gene_name": "Putative golgin subfamily A member 8D",
  "term_label": "cis-Golgi network",
  "term_id": "GO:0005801"
}